{
  "gene_symbol": "NPIPB7",
  "term_id": "UNKNOWN:0001",
  "gene": "UniProtKB:O75200",
  "gene_name": "Nuclear pore complex-interacting protein family member B7",
  "term_label": "Unknown molecular function"
}